{
  "gene_symbol": "CNOT4",
  "term_id": "GO:0016567",
  "term_label": "protein ubiquitination",
  "gene_name": "CCR4-NOT transcription complex subunit 4",
  "gene": "UniProtKB:O95628"
}